{
  "gene": "UniProtKB:Q32NC0",
  "gene_name": "UPF0711 protein C18orf21",
  "gene_symbol": "C18orf21",
  "term_label": "Unknown biological process",
  "term_id": "UNKNOWN:0002"
}